{
  "term_label": "Unknown biological process",
  "gene_symbol": "A0A1B0GTQ1",
  "term_id": "UNKNOWN:0002",
  "gene_name": "Uncharacterized protein",
  "gene": "UniProtKB:A0A1B0GTQ1"
}